{
  "gene_name": "Ran-binding protein 17",
  "gene": "UniProtKB:Q9H2T7",
  "term_id": "GO:0006611",
  "gene_symbol": "RANBP17",
  "term_label": "protein export from nucleus"
}